{
  "term_label": "cell surface receptor protein tyrosine kinase signaling pathway",
  "term_id": "GO:0007169",
  "gene_name": "NT-3 growth factor receptor",
  "gene": "UniProtKB:Q16288",
  "gene_symbol": "NTRK3"
}